{
  "gene_symbol": "ZNF609",
  "gene": "UniProtKB:O15014",
  "term_label": "nucleus",
  "term_id": "GO:0005634",
  "gene_name": "Zinc finger protein 609"
}